{
  "gene_symbol": "CFTR",
  "term_label": "water transport",
  "gene": "UniProtKB:P13569",
  "term_id": "GO:0006833",
  "gene_name": "Cystic fibrosis transmembrane conductance regulator"
}